methylenetetrahydrofolate reductase (NADH) activity [GO:0106312] (molecular function) Sources: RHEA:19821 Definition: Catalysis of the reaction: (6S)-5-methyl-5,6,7,8-tetrahydrofolate + NAD+ = (6R)-5,10-methylene-5,6,7,8-tetrahydrofolate + NADH + H+. Relationships: is a type of methylenetetrahydrofolate reductase [NAD(P)H] activity [GO:0004489]